violaceol II catabolic process [GO:1900592] (biological process) Definition: The chemical reactions and pathways resulting in the breakdown of violaceol II. Sources: GOC:TermGenie, GOC:di Also known as: violaceol II breakdown, violaceol II catabolism, violaceol II degradation Relationships: is_a GO:0019614; is a type of secondary metabolite catabolic process [GO:0090487]; is a type of violaceol II metabolic process [GO:1900591]; is a type of ether catabolic process [GO:1901502]